response to decreased oxygen levels [GO:0036293] (biological process) Relationships: is a type of response to oxygen levels [GO:0070482] Also known as: response to lowered oxygen levels Sources: GOC:al Definition: Any process that results in a change in state or activity of a cell or an organism (in terms of movement, secretion, enzyme production, gene expression, etc.) as a result of a stimulus reflecting a decline in the level of oxygen. Note: This term should be used when a decrease in oxygen levels is not considered a stress response. For a hypoxic stress response, consider instead 'response to hypoxia ; GO:0001666'. Subtypes: response to hypoxia [GO:0001666], GO:0034059, GO:0036294, response to oxygen-glucose deprivation [GO:0090649]